{
  "gene_name": "Cyclin-dependent kinase 5",
  "gene_symbol": "CDK5",
  "term_id": "GO:0004693",
  "gene": "UniProtKB:Q00535",
  "term_label": "cyclin-dependent protein serine/threonine kinase activity"
}